{
  "gene": "UniProtKB:Q6ZMT9",
  "term_id": "UNKNOWN:0002",
  "gene_name": "Death domain-containing protein 1",
  "term_label": "Unknown biological process",
  "gene_symbol": "DTHD1"
}